{
  "term_id": "GO:0005886",
  "term_label": "plasma membrane",
  "gene_name": "XK-related protein 6",
  "gene_symbol": "XKR6",
  "gene": "UniProtKB:Q5GH73"
}